{
  "gene": "UniProtKB:P11161",
  "gene_symbol": "EGR2",
  "gene_name": "E3 SUMO-protein ligase EGR2",
  "term_id": "GO:0005634",
  "term_label": "nucleus"
}